{
  "term_id": "GO:0070006",
  "gene": "UniProtKB:Q9UIQ6",
  "term_label": "metalloaminopeptidase activity",
  "gene_symbol": "LNPEP",
  "gene_name": "Leucyl-cystinyl aminopeptidase"
}